{
  "gene_name": "Calpain-13",
  "term_id": "GO:0004198",
  "gene": "UniProtKB:Q6MZZ7",
  "gene_symbol": "CAPN13",
  "term_label": "calcium-dependent cysteine-type endopeptidase activity"
}